{
  "gene_name": "N-alpha-acetyltransferase 80",
  "term_label": "cytoplasm",
  "gene": "UniProtKB:Q93015",
  "term_id": "GO:0005737",
  "gene_symbol": "NAA80"
}